positive regulation of pentose-phosphate shunt [GO:1905857] (biological process) Relationships: is a type of GO:0043456; is a type of positive regulation of purine nucleotide metabolic process [GO:1900544]; positively regulates GO:0006098 References: PMID:19015259 Sources: GOC:TermGenie, GO_REF:0000058 Definition: Any process that activates or increases the frequency, rate or extent of pentose-phosphate shunt.